{
  "term_id": "GO:0044716",
  "term_label": "8-oxo-GDP phosphatase activity",
  "gene_symbol": "NUDT18",
  "gene_name": "8-oxo-dGDP phosphatase NUDT18",
  "gene": "UniProtKB:Q6ZVK8"
}